ubiquitin activating enzyme complex [GO:0120123] (cellular component) Definition: A protein complex responsible for the catalysis of the reaction: E1 + ubiquitin + ATP--> E1-ubiquitin + AMP + PPi, where the E1-ubiquitin linkage is a thioester bond between the C-terminal glycine of Ub and a sulfhydryl side group of an E1 cysteine residue. This is the first step in a cascade of reactions in which ubiquitin is ultimately added to a protein substrate. Relationships: is a type of GO:0140535; is a type of catalytic complex [GO:1902494] Also known as: E1 complex, E1 ubiquitin-activating enzyme References: PMID:9545234 Sources: GOC:lnp